regulation of male germ cell proliferation [GO:2000254] (biological process) Subtypes: GO:2000255, GO:2000256 Sources: GOC:obol Relationships: is a type of regulation of germ cell proliferation [GO:1905936]; regulates male germ cell proliferation [GO:0002176] Definition: Any process that modulates the frequency, rate or extent of male germ cell proliferation.